{
  "term_label": "Unknown biological process",
  "gene_symbol": "ZMYM6",
  "gene": "UniProtKB:O95789",
  "term_id": "UNKNOWN:0002",
  "gene_name": "Zinc finger MYM-type protein 6"
}